{
  "term_id": "GO:0005634",
  "gene": "UniProtKB:Q9H707",
  "gene_name": "Zinc finger protein 552",
  "gene_symbol": "ZNF552",
  "term_label": "nucleus"
}